{
  "term_id": "UNKNOWN:0001",
  "gene_symbol": "IL1RAPL2",
  "gene_name": "X-linked interleukin-1 receptor accessory protein-like 2",
  "term_label": "Unknown molecular function",
  "gene": "UniProtKB:Q9NP60"
}